{
  "gene_name": "Calcium-binding and coiled-coil domain-containing protein 2",
  "gene": "UniProtKB:Q13137",
  "term_id": "GO:1901098",
  "term_label": "positive regulation of autophagosome maturation",
  "gene_symbol": "CALCOCO2"
}